elastic fiber assembly [GO:0048251] (biological process) Relationships: is a type of extracellular matrix assembly [GO:0085029]; is a type of supramolecular fiber organization [GO:0097435] Also known as: elastic fibre assembly, elastin fiber assembly, elastin fibre assembly Definition: Assembly of the extracellular matrix fibers that enables the matrix to recoil after transient stretching. References: PMID:10841810, PMID:12615674 Sources: GOC:jid